{
  "gene_symbol": "SLC7A6",
  "gene": "UniProtKB:Q92536",
  "term_label": "Unknown cellular component",
  "term_id": "UNKNOWN:0003",
  "gene_name": "Y+L amino acid transporter 2"
}